calcium sensitive guanylate cyclase activator activity [GO:0008048] (molecular function) Definition: Binds to and increases the activity of guanylate cyclase in response to a change in calcium ion concentration. Sources: GOC:mah Relationships: is a type of GO:0030250